{
  "gene_symbol": "TNKS2",
  "gene": "UniProtKB:Q9H2K2",
  "term_id": "GO:1904355",
  "gene_name": "Poly [ADP-ribose] polymerase tankyrase-2",
  "term_label": "positive regulation of telomere capping"
}